{
  "gene_name": "Polycomb group protein ASXL1",
  "gene": "UniProtKB:Q8IXJ9",
  "term_id": "GO:0009887",
  "term_label": "animal organ morphogenesis",
  "gene_symbol": "ASXL1"
}